regulation of proteasome assembly [GO:0090364] (biological process) Relationships: is a type of regulation of protein-containing complex assembly [GO:0043254]; regulates proteasome assembly [GO:0043248] Sources: GOC:dph, GOC:elh, GOC:tb Definition: Any process that modulates the rate, frequency, or extent of the aggregation, arrangement and bonding together of a mature, active proteasome complex.